{
  "term_label": "DNA topological change",
  "gene": "UniProtKB:P11387",
  "gene_name": "DNA topoisomerase 1",
  "term_id": "GO:0006265",
  "gene_symbol": "TOP1"
}